{
  "gene_name": "Ras-related protein Rab-3D",
  "gene_symbol": "RAB3D",
  "term_id": "GO:0003924",
  "gene": "UniProtKB:O95716",
  "term_label": "GTPase activity"
}